tartrate epimerase activity [GO:0050320] (molecular function) Definition: Catalysis of the reaction: L-tartrate = (2R,3S)-tartrate. Sources: EC:5.1.2.5, RHEA:22212 Also known as: tartaric racemase activity Relationships: is a type of racemase and epimerase activity, acting on hydroxy acids and derivatives [GO:0016856]